negative regulation of apoptotic process [GO:0043066] (biological process) Sources: GOC:jl, GOC:mtg_apoptosis Note: This term should only be used when it is not possible to determine which phase or subtype of the apoptotic process is negatively regulated by a gene product. Whenever detailed information is available, the more granular children terms should be used. Subtypes: negative regulation of muscle cell apoptotic process [GO:0010656], GO:0033033, negative regulation of glial cell apoptotic process [GO:0034351], negative regulation of neuron apoptotic process [GO:0043524], negative regulation of apoptotic process in bone marrow cell [GO:0071866], negative regulation of execution phase of apoptosis [GO:1900118], GO:1901693, negative regulation of epithelial cell apoptotic process [GO:1904036], negative regulation of myofibroblast cell apoptotic process [GO:1904521], negative regulation of fat cell apoptotic process [GO:1904650], negative regulation of apoptotic process involved in development [GO:1904746], negative regulation of leukocyte apoptotic process [GO:2000107], GO:2000270, GO:2000352, negative regulation of anoikis [GO:2000811], negative regulation of mesenchymal cell apoptotic process [GO:2001054], negative regulation of apoptotic signaling pathway [GO:2001234] Relationships: is a type of GO:0042981; is a type of GO:0043069; negatively regulates apoptotic process [GO:0006915] Also known as: anti-apoptosis, down regulation of apoptosis, down-regulation of apoptosis, downregulation of apoptosis, inhibition of apoptosis, negative regulation of apoptosis, apoptosis inhibitor activity, pro-survival Definition: Any process that stops, prevents, or reduces the frequency, rate or extent of cell death by apoptotic process.